toluene biosynthetic process [GO:0046252] (biological process) Definition: The chemical reactions and pathways resulting in the formation of toluene, a volatile monoaromatic hydrocarbon found in crude petroleum and petroleum products. Also known as: toluene anabolism, toluene biosynthesis, toluene formation, toluene synthesis Note: This term was reinstated from obsolete. Subtypes: anaerobic toluene biosynthetic process [GO:0046253] Relationships: is a type of toluene metabolic process [GO:0018970]; is a type of hydrocarbon biosynthetic process [GO:0120251] References: PMID:6508079 Sources: GOC:ai